{
  "gene_name": "G-protein coupled receptor family C group 6 member A",
  "term_label": "plasma membrane",
  "gene": "UniProtKB:Q5T6X5",
  "gene_symbol": "GPRC6A",
  "term_id": "GO:0005886"
}